{
  "term_label": "cytokine activity",
  "gene": "UniProtKB:Q00604",
  "term_id": "GO:0005125",
  "gene_symbol": "NDP",
  "gene_name": "Norrin"
}